{
  "term_label": "SOSS complex",
  "gene": "UniProtKB:Q9NRY2",
  "gene_symbol": "INIP",
  "term_id": "GO:0070876",
  "gene_name": "SOSS complex subunit C"
}